{
  "gene_name": "Synaptotagmin-10",
  "term_id": "GO:0061891",
  "term_label": "calcium ion sensor activity",
  "gene": "UniProtKB:Q6XYQ8",
  "gene_symbol": "SYT10"
}